transmembrane receptor protein serine/threonine kinase binding [GO:0070696] (molecular function) Definition: Binding to a receptor that spans a cell membrane and possesses protein serine/threonine kinase activity. Sources: GOC:BHF, GOC:mah Relationships: is_a receptor serine/threonine kinase binding [GO:0033612] Subtypes: activin receptor binding [GO:0070697], GO:0070700